negative regulation of lateral root development [GO:1901332] (biological process) Sources: GOC:TermGenie Relationships: is_a negative regulation of post-embryonic development [GO:0048581]; is a type of regulation of lateral root development [GO:2000023]; negatively regulates GO:0048527 Definition: Any process that stops, prevents or reduces the frequency, rate or extent of lateral root development. Also known as: down regulation of lateral root development, down-regulation of lateral root development, downregulation of lateral root development, inhibition of lateral root development